regulation of ribosomal large subunit export from nucleus [GO:2000203] (biological process) Relationships: is a type of regulation of ribosomal subunit export from nucleus [GO:2000200]; RO_0002211 ribosomal large subunit export from nucleus [GO:0000055] Sources: GOC:mah Definition: Any process that modulates the frequency, rate or extent of ribosomal large subunit export from nucleus. Subtypes: negative regulation of ribosomal large subunit export from nucleus [GO:2000204], positive regulation of ribosomal large subunit export from nucleus [GO:2000205] Also known as: regulation of ribosomal large subunit export from cell nucleus, regulation of ribosomal large subunit export out of nucleus, regulation of ribosomal large subunit transport from nucleus to cytoplasm, regulation of ribosomal large subunit-nucleus export, regulation of 50S ribosomal subunit export from nucleus, regulation of 60S ribosomal subunit export from nucleus